{
  "term_label": "Unknown biological process",
  "gene": "UniProtKB:P0DJI9",
  "term_id": "UNKNOWN:0002",
  "gene_symbol": "SAA2",
  "gene_name": "Serum amyloid A-2 protein"
}